{
  "gene_name": "PRAME family member 2",
  "term_label": "cytoplasm",
  "term_id": "GO:0005737",
  "gene_symbol": "PRAMEF2",
  "gene": "UniProtKB:O60811"
}